nucleic acid biosynthetic process [GO:0141187] (biological process) Sources: GOC:dph, GOC:tb Relationships: is a type of macromolecule biosynthetic process [GO:0009059]; is a type of GO:0034654; is a type of nucleic acid metabolic process [GO:0090304] Definition: The biosynthetic process resulting in the formation of a nucleic acid. Subtypes: GO:0032774, DNA biosynthetic process [GO:0071897] Note: This term should not be used for direct annotation. It should be possible to make a more specific annotation to one of the children of this term.